{
  "gene_name": "Solute carrier family 52, riboflavin transporter, member 3",
  "term_label": "riboflavin transmembrane transporter activity",
  "gene_symbol": "SLC52A3",
  "gene": "UniProtKB:Q9NQ40",
  "term_id": "GO:0032217"
}